maintenance of plastid location [GO:0051688] (biological process) Sources: GOC:ai, GOC:dph, GOC:tb Relationships: is a type of plastid localization [GO:0051644]; is_a maintenance of organelle location [GO:0051657] Also known as: maintenance of plastid localization Definition: Any process in which a plastid is maintained in a specific location within a cell and prevented from moving elsewhere.